response to nickel cation [GO:0010045] (biological process) Sources: GOC:sm Subtypes: GO:0071289 Definition: Any process that results in a change in state or activity of a cell or an organism (in terms of movement, secretion, enzyme production, gene expression, etc.) as a result of a nickel cation stimulus. Relationships: is a type of response to metal ion [GO:0010038] Also known as: response to nickel